{
  "term_id": "GO:0031146",
  "gene_symbol": "FBXW4",
  "term_label": "SCF-dependent proteasomal ubiquitin-dependent protein catabolic process",
  "gene": "UniProtKB:P57775",
  "gene_name": "F-box_WD repeat-containing protein 4"
}